{
  "term_id": "GO:0016558",
  "gene_name": "Peroxisome assembly protein 12",
  "gene_symbol": "PEX12",
  "gene": "UniProtKB:O00623",
  "term_label": "protein import into peroxisome matrix"
}